{
  "gene": "UniProtKB:P09237",
  "term_label": "extracellular space",
  "term_id": "GO:0005615",
  "gene_name": "Matrilysin",
  "gene_symbol": "MMP7"
}